sperm incapacitation [GO:0046694] (biological process) Definition: The process in which the use of stored sperm from the first-mating male is inhibited by the seminal fluid of subsequently mating males. Relationships: is a type of sperm competition [GO:0046692] References: PMID:10440373